ajugose biosynthetic process using galactinol:raffinose galactosyltransferase [GO:0033537] (biological process) Definition: The chemical reactions and pathways resulting in the formation of ajugose, the hexasaccharide beta-D-fructofuranosyl alpha-D-galactopyranosyl-(1->6)-alpha-D-galactopyranosyl-(1->6)-alpha-D-galactopyranosyl-(1->6)-alpha-D-galactopyranosyl-(1->6)-alpha-D-glucopyranoside, by a pathway in which galactinol:raffinose galactosyltransferase catalyzes chain elongation by transferring the alpha-galactosyl residue of galactinol to the oligosaccharide. Sources: GOC:mah, MetaCyc:PWY-5342 Also known as: ajugose anabolism using galactinol:raffinose galactosyltransferase, ajugose biosynthesis using galactinol:raffinose galactosyltransferase, ajugose formation using galactinol:raffinose galactosyltransferase, ajugose synthesis using galactinol:raffinose galactosyltransferase Relationships: is a type of GO:0033536